erythrocyte homeostasis [GO:0034101] (biological process) Also known as: RBC homeostasis, red blood cell homeostasis Definition: Any process of regulating the production and elimination of erythrocytes within an organism. References: PMID:10694114, PMID:14754397 Sources: GOC:add Relationships: is a type of myeloid cell homeostasis [GO:0002262]